{
  "gene": "UniProtKB:P0DOY2",
  "term_label": "IgG immunoglobulin complex",
  "term_id": "GO:0071735",
  "gene_name": "Immunoglobulin lambda constant 2",
  "gene_symbol": "IGLC2"
}